cone telodendria [GO:0120209] (cellular component) Definition: Cone telodendria are projections that originate from the cone pedicle and form gap junctions with other photoreceptors within the outer plexiform layer of the retina. References: PMID:29127712 Sources: GOC:cvs, GOC:krc Relationships: is a type of telodendria [GO:0120208]